antimicrobial peptide secretion [GO:0002776] (biological process) Regulation: regulated by GO:0002794; negatively regulated by GO:0002795; positively regulated by positive regulation of antimicrobial peptide secretion [GO:0002796] References: PMID:11807545, PMID:15638771 Sources: GOC:add, ISBN:0781735149 Definition: The regulated release of an antimicrobial peptide from a cell or a tissue. Such peptides may have protective properties against bacteria, fungi, viruses, or protozoa. Subtypes: GO:0002779, antifungal peptide secretion [GO:0002782] Relationships: is a type of peptide secretion [GO:0002790]; is part of antimicrobial peptide production [GO:0002775]